{
  "gene": "UniProtKB:P20248",
  "term_label": "cyclin A2-CDK2 complex",
  "gene_symbol": "CCNA2",
  "gene_name": "Cyclin-A2",
  "term_id": "GO:0097124"
}